{
  "term_id": "GO:0030154",
  "gene_symbol": "NANOG",
  "gene_name": "Homeobox protein NANOG",
  "term_label": "cell differentiation",
  "gene": "UniProtKB:Q9H9S0"
}